{
  "term_id": "GO:0043137",
  "gene_symbol": "RNASEH1",
  "gene_name": "Ribonuclease H1",
  "term_label": "DNA replication, removal of RNA primer",
  "gene": "UniProtKB:O60930"
}